{
  "term_label": "nucleus",
  "term_id": "GO:0005634",
  "gene": "UniProtKB:Q14004",
  "gene_symbol": "CDK13",
  "gene_name": "Cyclin-dependent kinase 13"
}